{
  "gene_symbol": "YIPF4",
  "gene_name": "Protein YIPF4",
  "term_label": "trans-Golgi network",
  "gene": "UniProtKB:Q9BSR8",
  "term_id": "GO:0005802"
}